{
  "gene_name": "Protein kinase C epsilon type",
  "gene": "UniProtKB:Q02156",
  "term_label": "Unknown cellular component",
  "gene_symbol": "PRKCE",
  "term_id": "UNKNOWN:0003"
}